{
  "term_id": "GO:0044183",
  "gene_symbol": "HSPA1B",
  "gene": "UniProtKB:P0DMV9",
  "term_label": "protein folding chaperone",
  "gene_name": "Heat shock 70 kDa protein 1B"
}